{
  "gene_name": "Gamma-enolase",
  "term_id": "GO:0006096",
  "gene_symbol": "ENO2",
  "gene": "UniProtKB:P09104",
  "term_label": "glycolytic process"
}